{
  "term_id": "GO:0005109",
  "gene_name": "Segment polarity protein dishevelled homolog DVL-1",
  "gene": "UniProtKB:O14640",
  "term_label": "frizzled binding",
  "gene_symbol": "DVL1"
}